posterior neuropore closure [GO:0021507] (biological process) Relationships: is a type of morphogenesis of embryonic epithelium [GO:0016331]; is a type of cell-cell adhesion involved in neural tube closure [GO:0060608]; is part of neuropore closure [GO:0021995] Sources: GOC:cls, GOC:dgh, GOC:dph, GOC:jid, GO_REF:0000021 Definition: The joining together of the neural folds of the caudal opening of the neural tube. The posterior neuropore appears before the process of neural tube closure is complete.